{
  "term_label": "positive regulation of transcription by RNA polymerase II",
  "term_id": "GO:0045944",
  "gene_symbol": "IKBKB",
  "gene": "UniProtKB:O14920",
  "gene_name": "Inhibitor of nuclear factor kappa-B kinase subunit beta"
}